{
  "term_label": "negative regulation of programmed cell death",
  "gene": "UniProtKB:Q9NS93",
  "term_id": "GO:0043069",
  "gene_symbol": "TM7SF3",
  "gene_name": "Transmembrane 7 superfamily member 3"
}